neurotrophin receptor binding [GO:0005165] (molecular function) Subtypes: nerve growth factor receptor binding [GO:0005163], neurotrophin p75 receptor binding [GO:0005166], neurotrophin TRK receptor binding [GO:0005167], brain-derived neurotrophic factor receptor binding [GO:0031546] Definition: Binding to a neurotrophin receptor. Relationships: is a type of GO:0005126 Also known as: neurotrophin, neurotrophin receptor ligand Sources: GOC:ai